{
  "gene": "UniProtKB:Q9NP90",
  "term_id": "UNKNOWN:0001",
  "term_label": "Unknown molecular function",
  "gene_symbol": "RAB9B",
  "gene_name": "Ras-related protein Rab-9B"
}